{
  "gene": "UniProtKB:P12757",
  "term_label": "cytoplasm",
  "gene_symbol": "SKIL",
  "term_id": "GO:0005737",
  "gene_name": "Ski-like protein"
}